{
  "term_id": "GO:0003899",
  "gene_name": "DNA-directed primase_polymerase protein",
  "term_label": "DNA-directed RNA polymerase activity",
  "gene": "UniProtKB:Q96LW4",
  "gene_symbol": "PRIMPOL"
}